flippase activity [GO:0140327] (molecular function) Note: Nomenclature note. Flippases and floppases are ATP-dependent transbilayer lipid translocators. According to an extensively used, though not universal, nomenclature, they catalyze lipid transfer towards the inward monolayer (flippases) or towards the outward monolayer (floppases). Scramblases are ATP-independent, non-selective, inducing non-specific transbilayer movements across the membrane. The direction of the translocation should be taken into account for annotation (from the exoplasmic to the cytosolic leaflet of a membrane). Also known as: flippase activity (exoplasmic to cytosolic leaflet) Relationships: is a type of ATPase-coupled intramembrane lipid transporter activity [GO:0140326] Definition: Catalysis of the movement of lipids from the exoplasmic to the cytosolic leaflet of a membrane, using energy from the hydrolysis of ATP. Subtypes: aminophospholipid flippase activity [GO:0015247], glycerophospholipid flippase activity [GO:0140333], GO:0140351 References: PMID:20043909, PMID:25284293 Sources: Wikipedia:Flippase